nipple development [GO:0060618] (BP) Sources: GOC:dph Definition: The progression of the nipple over time, from its formation to the mature structure. The nipple is a part of the mammary gland that protrudes from the surface ectoderm. Relationships: is a type of anatomical structure development [GO:0048856]; is part of mammary gland development [GO:0030879]